{
  "gene_symbol": "TEAD2",
  "gene_name": "Transcriptional enhancer factor TEF-4",
  "term_label": "RNA polymerase II cis-regulatory region sequence-specific DNA binding",
  "term_id": "GO:0000978",
  "gene": "UniProtKB:Q15562"
}